esterosome [GO:0033117] (cellular component) Definition: A vesicle filled with crystalline protein that shows sequence similarities with various esterases. Relationships: is a type of cytoplasmic vesicle [GO:0031410] References: PMID:2307702 Sources: GOC:ecd